{
  "gene_symbol": "BTNL3",
  "gene": "UniProtKB:Q6UXE8",
  "term_label": "signaling receptor binding",
  "term_id": "GO:0005102",
  "gene_name": "Butyrophilin-like protein 3"
}